{
  "term_id": "GO:0016477",
  "gene_symbol": "CDH17",
  "term_label": "cell migration",
  "gene": "UniProtKB:Q12864",
  "gene_name": "Cadherin-17"
}